negative regulation of leukocyte differentiation [GO:1902106] (biological process) Sources: GOC:TermGenie, GOC:add Subtypes: GO:0002762, negative regulation of lymphocyte differentiation [GO:0045620], negative regulation of dendritic cell differentiation [GO:2001199] Definition: Any process that stops, prevents or reduces the frequency, rate or extent of leukocyte differentiation. Also known as: down regulation of immune cell differentiation, down regulation of leucocyte differentiation, down regulation of leukocyte differentiation, down-regulation of immune cell differentiation, down-regulation of leucocyte differentiation, down-regulation of leukocyte differentiation, downregulation of immune cell differentiation, downregulation of leucocyte differentiation, downregulation of leukocyte differentiation, negative regulation of immune cell differentiation, negative regulation of leucocyte differentiation, inhibition of immune cell differentiation, inhibition of leucocyte differentiation, inhibition of leukocyte differentiation Relationships: is a type of regulation of leukocyte differentiation [GO:1902105]; is a type of GO:1903707; negatively regulates leukocyte differentiation [GO:0002521]